{
  "gene": "UniProtKB:Q7Z713",
  "gene_symbol": "ANKRD37",
  "term_label": "Unknown biological process",
  "gene_name": "Ankyrin repeat domain-containing protein 37",
  "term_id": "UNKNOWN:0002"
}